{
  "gene_symbol": "PNPLA6",
  "term_id": "GO:0005783",
  "term_label": "endoplasmic reticulum",
  "gene": "UniProtKB:Q8IY17",
  "gene_name": "Patatin-like phospholipase domain-containing protein 6"
}